{
  "gene_symbol": "DMRT3",
  "term_id": "GO:0006357",
  "gene_name": "Doublesex- and mab-3-related transcription factor 3",
  "term_label": "regulation of transcription by RNA polymerase II",
  "gene": "UniProtKB:Q9NQL9"
}